{
  "term_id": "GO:0005415",
  "gene_symbol": "SLC28A2",
  "term_label": "nucleoside:sodium symporter activity",
  "gene": "UniProtKB:O43868",
  "gene_name": "Sodium_nucleoside cotransporter 2"
}